{
  "term_label": "Unknown cellular component",
  "gene_symbol": "C6orf50",
  "gene_name": "Putative uncharacterized protein C6orf50",
  "term_id": "UNKNOWN:0003",
  "gene": "UniProtKB:Q9HD87"
}